{
  "term_id": "GO:0005802",
  "gene_symbol": "CNST",
  "gene_name": "Consortin",
  "gene": "UniProtKB:Q6PJW8",
  "term_label": "trans-Golgi network"
}